{
  "gene_name": "Interferon regulatory factor 1",
  "term_label": "DNA-binding transcription factor activity, RNA polymerase II-specific",
  "gene": "UniProtKB:P10914",
  "gene_symbol": "IRF1",
  "term_id": "GO:0000981"
}